{
  "gene": "UniProtKB:Q9BXF3",
  "gene_name": "Chromatin remodeling regulator CECR2",
  "term_label": "CERF complex",
  "gene_symbol": "CECR2",
  "term_id": "GO:0090537"
}